{
  "term_id": "GO:0000149",
  "gene_name": "Synaptotagmin-7",
  "term_label": "SNARE binding",
  "gene_symbol": "SYT7",
  "gene": "UniProtKB:O43581"
}